eukaryotic initiation factor 4G binding [GO:0031370] (molecular function) Relationships: is a type of translation initiation factor binding [GO:0031369] Sources: GOC:mah Also known as: eIF4G binding Definition: Binding to eukaryotic initiation factor 4G, a polypeptide factor involved in the initiation of ribosome-mediated translation.